cellular response to transforming growth factor beta stimulus [GO:0071560] (BP) Definition: Any process that results in a change in state or activity of a cell (in terms of movement, secretion, enzyme production, gene expression, etc.) as a result of a transforming growth factor beta stimulus. Relationships: is a type of cellular response to growth factor stimulus [GO:0071363]; is a type of response to transforming growth factor beta [GO:0071559] References: PMID:15451575 Sources: GOC:ecd Also known as: cellular response to TGF-beta stimulus, cellular response to TGFbeta stimulus Regulation: regulated by regulation of cellular response to transforming growth factor beta stimulus [GO:1903844]; negatively regulated by negative regulation of cellular response to transforming growth factor beta stimulus [GO:1903845]; positively regulated by positive regulation of cellular response to transforming growth factor beta stimulus [GO:1903846]